L-3-cyanoalanine synthase activity [GO:0050017] (molecular function) Sources: EC:4.4.1.9, MetaCyc:L-3-CYANOALANINE-SYNTHASE-RXN Also known as: L-cysteine hydrogen-sulfide-lyase (adding HCN), L-cysteine hydrogen-sulfide-lyase (adding hydrogen cyanide; L-3-cyanoalanine-forming), beta-cyano-L-alanine synthase activity, beta-cyanoalanine synthase activity, beta-cyanoalanine synthetase activity Definition: Catalysis of the reaction: L-cysteine + HCN = sulfide + L-3-cyanoalanine. Relationships: is a type of GO:0016846